{
  "gene_name": "TP53-target gene 5 protein",
  "term_label": "Unknown biological process",
  "gene": "UniProtKB:Q9Y2B4",
  "term_id": "UNKNOWN:0002",
  "gene_symbol": "TP53TG5"
}